oxidoreductase activity, acting on phosphorus or arsenic in donors [GO:0030613] (molecular function) Relationships: is_a oxidoreductase activity [GO:0016491] Also known as: oxidoreductase activity, acting on phosphorus or arsenic in donors, with other acceptors Sources: EC:1.20.-.- Subtypes: arsenate reductase activity [GO:0030611], oxidoreductase activity, acting on phosphorus or arsenic in donors, disulfide as acceptor [GO:0030614], oxidoreductase activity, acting on phosphorus or arsenic in donors, with NAD(P)+ as acceptor [GO:0050499], GO:0052882 Definition: Catalysis of an oxidation-reduction (redox) reaction in which a phosphorus- or arsenic-containing group acts as a hydrogen or electron donor and reduces a hydrogen or electron acceptor.